glycerol channel activity [GO:0015254] (molecular function) Definition: Enables the energy-independent facilitated diffusion of glycerol through a transmembrane aqueous pore or channel. Relationships: is a type of glycerol transmembrane transporter activity [GO:0015168]; is a type of channel activity [GO:0015267] Sources: GOC:mtg_transport, ISBN:0815340729